{
  "gene_symbol": "METTL3",
  "term_label": "RNA N6-methyladenosine methyltransferase complex",
  "gene_name": "N6-adenosine-methyltransferase catalytic subunit",
  "gene": "UniProtKB:Q86U44",
  "term_id": "GO:0036396"
}